{
  "gene": "UniProtKB:P19237",
  "gene_symbol": "TNNI1",
  "gene_name": "Troponin I, slow skeletal muscle",
  "term_label": "Unknown molecular function",
  "term_id": "UNKNOWN:0001"
}